{
  "term_id": "UNKNOWN:0003",
  "term_label": "Unknown cellular component",
  "gene": "UniProtKB:Q9H993",
  "gene_symbol": "ARMT1",
  "gene_name": "Damage-control phosphatase ARMT1"
}